{
  "term_label": "G protein-coupled photoreceptor activity",
  "gene_name": "Melanopsin",
  "term_id": "GO:0008020",
  "gene": "UniProtKB:Q9UHM6",
  "gene_symbol": "OPN4"
}